frontal suture morphogenesis [GO:0060364] (biological process) Definition: The process in which the frontal suture is generated and organized. Sources: GOC:dph, GOC:sl Also known as: interfrontal suture morphogenesis Relationships: is_a cranial suture morphogenesis [GO:0060363]